nitric-oxide synthase binding [GO:0050998] (molecular function) Relationships: is a type of enzyme binding [GO:0019899] Definition: Binding to nitric-oxide synthase. Sources: GOC:ai Also known as: NOS binding